catalytic activity, acting on a nucleic acid [GO:0140640] (molecular function) Definition: Catalytic activity that acts to modify a nucleic acid. Relationships: is a type of catalytic activity [GO:0003824] Subtypes: GO:0004386, nuclease activity [GO:0004518], catalytic activity, acting on DNA [GO:0140097], GO:0140098, annealing activity [GO:0140666], GO:0160225 Sources: GOC:pg